etioplast organization [GO:0009662] (biological process) Sources: GOC:jid Also known as: etioplast organisation, etioplast organization and biogenesis Relationships: is a type of plastid organization [GO:0009657] Definition: A process that is carried out at the cellular level which results in the assembly, arrangement of constituent parts, or disassembly of an etioplast. An etioplast is a plastid arrested in the development of chloroplasts from proplastids due to absence of light or low light conditions.